nuclear protein quality control by the ubiquitin-proteasome system [GO:0071630] (biological process) Definition: A protein quality control pathway that results in the breakdown of misfolded, damaged or unassembled proteins via a mechanism in which the proteins are ubiquitinated, and then targeted to nuclear proteasomes for degradation. References: PMID:20080635, PMID:21211726 Relationships: is_a GO:0006515; is a type of proteasome-mediated ubiquitin-dependent protein catabolic process [GO:0043161]; BFO_0000050 cellular response to misfolded protein [GO:0071218] Also known as: nucleus-associated proteasomal ubiquitin-dependent protein breakdown, nucleus-associated proteasomal ubiquitin-dependent protein catabolism, nucleus-associated proteasomal ubiquitin-dependent protein degradation, ubiquitin-dependent catabolism of misfolded proteins by nucleus-associated proteasome Subtypes: GO:0180027